{
  "gene_symbol": "NUDT3",
  "term_label": "nucleus",
  "gene_name": "Diphosphoinositol polyphosphate phosphohydrolase 1",
  "term_id": "GO:0005634",
  "gene": "UniProtKB:O95989"
}